{
  "gene_name": "T cell receptor alpha variable 6",
  "gene": "UniProtKB:A0A075B6T7",
  "gene_symbol": "TRAV6",
  "term_label": "Unknown cellular component",
  "term_id": "UNKNOWN:0003"
}